disruption of cellular anatomical structure in another organism [GO:0140975] (biological process) Relationships: is a type of GO:0141060 Also known as: disruption of cellular component of another organism Subtypes: disruption of plasma membrane integrity in another organism [GO:0051673] Sources: GOC:pg Definition: The disruption of a cellular component of another organism, leading to damage or temporary subversion of that structure. In some cases this can cause malfunctioning of the cells and death of the target organism.